{
  "gene_symbol": "SLC6A6",
  "gene": "UniProtKB:P31641",
  "term_id": "GO:0035725",
  "term_label": "sodium ion transmembrane transport",
  "gene_name": "Sodium- and chloride-dependent taurine transporter"
}